thyroid hormone receptor signaling pathway [GO:0002154] (biological process) Definition: A nuclear receptor-mediated signaling pathway initiated by a thyroid hormone  binding to an intracellular receptor of the nuclear receptor protein family, and ending with regulation of a downstream cellular process, e.g. transcription. Sources: GOC:hjd Also known as: thyroid hormone mediated signalling pathway Relationships: is a type of hormone-mediated signaling pathway [GO:0009755]; is a type of nuclear receptor-mediated signaling pathway [GO:0141193] Regulation: regulated by regulation of thyroid hormone receptor signaling pathway [GO:0002155]; negatively regulated by negative regulation of thyroid hormone receptor signaling pathway [GO:0002156]; positively regulated by positive regulation of thyroid hormone receptor signaling pathway [GO:0002157]